{
  "term_id": "UNKNOWN:0002",
  "gene_name": "Immunoglobulin-like domain-containing receptor 1",
  "term_label": "Unknown biological process",
  "gene_symbol": "ILDR1",
  "gene": "UniProtKB:Q86SU0"
}